methane biosynthetic process from carbon monoxide [GO:2001134] (biological process) Relationships: is a type of methanogenesis [GO:0015948] Definition: The chemical reactions and pathways resulting in the formation of a methane from a carbon monoxide. Regulation: regulated by regulation of methane biosynthetic process from carbon monoxide [GO:1900336]; negatively regulated by GO:1900337; positively regulated by positive regulation of methane biosynthetic process from carbon monoxide [GO:1900338] Sources: GOC:mengo_curators